heme import into cell [GO:0140420] (biological process) Definition: The directed movement of a heme from outside of a cell into a cell. This may occur via transport across the plasma membrane or via endocytosis. References: PMID:28193844 Also known as: heme assimilation Relationships: is a type of GO:0015886; is_a iron import into cell [GO:0033212] Subtypes: endocytic heme import into cell [GO:0140421], GO:1904334